{
  "gene": "UniProtKB:A8MXV6",
  "gene_name": "CMT1A duplicated region transcript 15 protein-like protein",
  "gene_symbol": "CDRT15L2",
  "term_label": "Unknown molecular function",
  "term_id": "UNKNOWN:0001"
}